Isw1a complex [GO:0036436] (cellular component) References: PMID:12482963 Sources: GOC:jd Definition: An Isw1 complex that binds DNA and has nucleosome-stimulated ATPase activity. In S. cerevisiae, contains an Isw1p ATPase subunit in complex with Ioc3p. Relationships: is a type of Isw1 complex [GO:0016587]